{
  "term_label": "Unknown biological process",
  "gene_symbol": "ANKDD1B",
  "term_id": "UNKNOWN:0002",
  "gene": "UniProtKB:A6NHY2",
  "gene_name": "Ankyrin repeat and death domain-containing protein 1B"
}